uridine metabolic process [GO:0046108] (biological process) Relationships: is a type of GO:0046131 Also known as: uridine metabolism Sources: GOC:go_curators Subtypes: uridine catabolic process [GO:0006218], uridine biosynthetic process [GO:0046109] Definition: The chemical reactions and pathways involving uridine, uracil riboside, a ribonucleoside very widely distributed but occurring almost entirely as phosphoric esters in ribonucleotides and ribonucleic acids.